4-hydroxybenzoate 3-monooxygenase [NAD(P)H] activity [GO:0018671] (molecular function) Definition: Catalysis of the reaction: 4-hydroxybenzoate + NAD(P)H + H+ + O2 = 3,4-dihydroxybenzoate + NAD(P)+ + H2O. Subtypes: GO:0106355, 4-hydroxybenzoate 3-monooxygenase (NADPH) activity [GO:0106356] Also known as: 4-hydroxybenzoate 3-hydroxylase activity, 4-hydroxybenzoate 3-monooxygenase (reduced nicotinamide adenine dinucleotide (phosphate)), 4-hydroxybenzoate,NAD(P)H:oxygen oxidoreductase (3-hydroxylating), 4-hydroxybenzoate-3-hydroxylase activity Relationships: is a type of oxidoreductase activity, acting on paired donors, with incorporation or reduction of molecular oxygen, NAD(P)H as one donor, and incorporation of one atom of oxygen [GO:0016709] Sources: EC:1.14.13.33